TFIIF-class transcription factor complex binding [GO:0001096] (molecular function) Relationships: is a type of RNA polymerase II general transcription initiation factor binding [GO:0001091]; is a type of protein-containing complex binding [GO:0044877] References: PMID:16858867 Sources: GOC:krc Also known as: TFIIF-class transcription factor binding Definition: Binding to a general RNA polymerase II transcription factor belonging to the TFIIF complex, one of the factors involved in formation of the preinitiation complex (PIC) by RNA polymerase II.